{
  "term_label": "nucleus",
  "gene_name": "Zinc finger protein 582",
  "gene_symbol": "ZNF582",
  "gene": "UniProtKB:Q96NG8",
  "term_id": "GO:0005634"
}